{
  "gene_name": "Nuclear receptor corepressor 2",
  "gene": "UniProtKB:Q9Y618",
  "gene_symbol": "NCOR2",
  "term_label": "chromatin",
  "term_id": "GO:0000785"
}